{
  "term_label": "SREBP-SCAP-Insig complex",
  "gene_name": "Insulin-induced gene 2 protein",
  "gene": "UniProtKB:Q9Y5U4",
  "gene_symbol": "INSIG2",
  "term_id": "GO:0032937"
}